{
  "gene_symbol": "CCDC57",
  "gene_name": "Coiled-coil domain-containing protein 57",
  "term_id": "GO:0005814",
  "gene": "UniProtKB:Q2TAC2",
  "term_label": "centriole"
}